{
  "gene_symbol": "KIF21A",
  "gene": "UniProtKB:Q7Z4S6",
  "gene_name": "Kinesin-like protein KIF21A",
  "term_id": "GO:0005874",
  "term_label": "microtubule"
}